trigeminal ganglion maturation [GO:0061557] (biological process) Definition: A developmental process, independent of morphogenetic (shape) change, that is required for a trigeminal ganglion to attain its fully functional state. Also known as: trigeminal ganglia maturation Relationships: is a type of GO:0061558; is part of trigeminal nerve maturation [GO:0021635]; BFO_0000050 trigeminal ganglion development [GO:0061551] Sources: GOC:dph